{
  "term_id": "GO:0006355",
  "gene_symbol": "SBNO1",
  "gene_name": "Protein strawberry notch homolog 1",
  "gene": "UniProtKB:A3KN83",
  "term_label": "regulation of DNA-templated transcription"
}